{
  "gene": "UniProtKB:P14854",
  "gene_name": "Cytochrome c oxidase subunit 6B1",
  "gene_symbol": "COX6B1",
  "term_label": "mitochondrion",
  "term_id": "GO:0005739"
}